{
  "term_id": "GO:0006357",
  "gene_name": "Kruppel-like factor 18",
  "gene_symbol": "KLF18",
  "term_label": "regulation of transcription by RNA polymerase II",
  "gene": "UniProtKB:A0A0U1RQI7"
}